protein-phosphocysteine-galactitol-phosphotransferase system transporter activity [GO:0090584] (molecular function) Relationships: is a type of protein-phosphocysteine-sugar phosphotransferase activity [GO:0090563] Definition: Catalysis of the PEP-dependent, phosphoryl transfer-driven transport of substances across a membrane. The transport happens by catalysis of the reaction: protein S-phosphocysteine + galactitol(out) = protein cysteine + galactitol-6-phosphate(in). References: PMID:8955298